ventricular zone neuroblast division [GO:0021847] (biological process) Relationships: is a type of forebrain ventricular zone progenitor cell division [GO:0021869]; is a type of forebrain neuroblast division [GO:0021873] References: PMID:12626695 Sources: GOC:cls, GOC:dgh, GOC:dph, GOC:jid, GO_REF:0000021 Also known as: neuroblast division in ventricular zone Definition: The proliferation of neuroblasts in the ventricular zone of the cerebral cortex. The neuronal progenitors of these cells will migrate radially.